regulation of strand invasion [GO:0060542] (biological process) Definition: Any process that modulates the rate, frequency or extent of strand invasion. Strand invasion is the process in which the nucleoprotein complex (composed of the broken single-strand DNA and the recombinase) searches and identifies a region of homology in intact duplex DNA. The broken single-strand DNA displaces the like strand and forms Watson-Crick base pairs with its complement, forming a duplex in which each strand is from one of the two recombining DNA molecules. Relationships: is a type of regulation of DNA metabolic process [GO:0051052]; regulates DNA strand invasion [GO:0042148] Sources: GOC:dph, GOC:tb Subtypes: negative regulation of strand invasion [GO:0060543], positive regulation of strand invasion [GO:0098530]